immune complex clearance by erythrocytes [GO:0002435] (biological process) Definition: The process of immune complex clearance by erythrocytes. The process often starts with binding of complement receptor 1 (CR1) on the surface of erythrocytes to a complement coated immune complex. The complex bound to erythrocyte CR1 is then transported to the liver or spleen where it is presented to phagocytes. The process ends when the complex is removed from CR1, allowing the erythrocyte to return to general circulation. References: PMID:11414352, PMID:24022490 Sources: GOC:add Also known as: immune complex clearance by RBCs, immune complex clearance by red blood cells Relationships: is a type of immune complex clearance [GO:0002434]